{
  "term_id": "UNKNOWN:0002",
  "gene": "UniProtKB:Q96M34",
  "gene_symbol": "TEX55",
  "term_label": "Unknown biological process",
  "gene_name": "Testis-specific expressed protein 55"
}